{
  "gene": "UniProtKB:Q6PEW0",
  "gene_symbol": "PRSS54",
  "gene_name": "Inactive serine protease 54",
  "term_label": "proteolysis",
  "term_id": "GO:0006508"
}